{
  "gene": "UniProtKB:Q9H819",
  "gene_symbol": "DNAJC18",
  "term_id": "GO:0030544",
  "gene_name": "DnaJ homolog subfamily C member 18",
  "term_label": "Hsp70 protein binding"
}